{
  "gene_name": "Interleukin-13 receptor subunit alpha-2",
  "term_id": "GO:0019221",
  "gene": "UniProtKB:Q14627",
  "gene_symbol": "IL13RA2",
  "term_label": "cytokine-mediated signaling pathway"
}